{
  "gene_symbol": "CCL11",
  "gene_name": "Eotaxin",
  "gene": "UniProtKB:P51671",
  "term_id": "GO:0061844",
  "term_label": "antimicrobial humoral immune response mediated by antimicrobial peptide"
}